negative regulation of small GTPase mediated signal transduction [GO:0051058] (biological process) Also known as: down regulation of small GTPase mediated signal transduction, down-regulation of small GTPase mediated signal transduction, downregulation of small GTPase mediated signal transduction, negative regulation of small GTPase-mediated signal transduction, inhibition of small GTPase mediated signal transduction Definition: Any process that stops, prevents, or reduces the frequency, rate or extent of small GTPase mediated signal transduction. Relationships: is a type of regulation of small GTPase mediated signal transduction [GO:0051056]; is_a negative regulation of intracellular signal transduction [GO:1902532]; negatively regulates GO:0007264 Sources: GOC:ai Subtypes: negative regulation of septation initiation signaling [GO:0031030], negative regulation of ARF protein signal transduction [GO:0032013], negative regulation of Rac protein signal transduction [GO:0035021], negative regulation of Rho protein signal transduction [GO:0035024], negative regulation of Ras protein signal transduction [GO:0046580]